{
  "gene": "UniProtKB:P46934",
  "gene_name": "E3 ubiquitin-protein ligase NEDD4",
  "gene_symbol": "NEDD4",
  "term_id": "GO:0031175",
  "term_label": "neuron projection development"
}